{
  "gene_name": "SMAD5 antisense gene protein 1",
  "gene_symbol": "SMAD5-AS1",
  "term_id": "UNKNOWN:0001",
  "term_label": "Unknown molecular function",
  "gene": "UniProtKB:Q9Y6J3"
}